{
  "term_label": "regulation of transcription by RNA polymerase II",
  "gene_name": "N-myc proto-oncogene protein",
  "term_id": "GO:0006357",
  "gene_symbol": "MYCN",
  "gene": "UniProtKB:P04198"
}